{
  "gene_symbol": "ELK3",
  "gene": "UniProtKB:P41970",
  "term_id": "GO:0005634",
  "gene_name": "ETS domain-containing protein Elk-3",
  "term_label": "nucleus"
}